{
  "gene": "UniProtKB:P47756",
  "gene_symbol": "CAPZB",
  "term_label": "Unknown biological process",
  "term_id": "UNKNOWN:0002",
  "gene_name": "F-actin-capping protein subunit beta"
}